{
  "gene_symbol": "RAB35",
  "term_id": "GO:0010008",
  "term_label": "endosome membrane",
  "gene": "UniProtKB:Q15286",
  "gene_name": "Ras-related protein Rab-35"
}